diphthine-ammonia ligase activity [GO:0017178] (molecular function) Definition: Catalysis of the reaction: ATP + diphthine + NH4 = ADP + diphthamide + H+ + phosphate. Sources: EC:6.3.1.14, RHEA:19753 Also known as: diphthamide synthase activity, diphthamide synthetase activity, diphthine:ammonia ligase (ADP-forming) Relationships: is a type of GO:0016880